{
  "term_label": "Unknown molecular function",
  "gene": "UniProtKB:Q9UPX0",
  "term_id": "UNKNOWN:0001",
  "gene_symbol": "IGSF9B",
  "gene_name": "Protein turtle homolog B"
}